{
  "term_label": "extracellular matrix",
  "gene": "UniProtKB:Q92954",
  "gene_symbol": "PRG4",
  "gene_name": "Proteoglycan 4",
  "term_id": "GO:0031012"
}